{
  "gene_symbol": "TCEAL3",
  "term_label": "Unknown biological process",
  "term_id": "UNKNOWN:0002",
  "gene_name": "Transcription elongation factor A protein-like 3",
  "gene": "UniProtKB:Q969E4"
}